{
  "gene_name": "Envoplakin-like protein",
  "term_id": "UNKNOWN:0003",
  "gene": "UniProtKB:A8MZ36",
  "term_label": "Unknown cellular component",
  "gene_symbol": "EVPLL"
}